myo-inositol hexakisphosphate transport [GO:0033272] (biological process) Relationships: is a type of organic anion transport [GO:0015711]; is a type of myo-inositol phosphate transport [GO:0033271] Also known as: phytate transport Definition: The directed movement of myo-inositol hexakisphosphate into, out of or within a cell, or between cells, by means of some agent such as a transporter or pore. Sources: GOC:mah